{
  "gene_symbol": "KRTAP12-2",
  "term_label": "Unknown biological process",
  "term_id": "UNKNOWN:0002",
  "gene_name": "Keratin-associated protein 12-2",
  "gene": "UniProtKB:P59991"
}